copper ion import across plasma membrane [GO:0098705] (biological process) Sources: GOC:dos Definition: The directed movement of copper ions from outside of a cell, across the plasma membrane and into the cytosol. Relationships: is_a GO:0015679; is a type of inorganic cation import across plasma membrane [GO:0098659] Also known as: copper cation import into cell, copper ion import into cell, high affinity copper ion transport, high affinity copper transport, high-affinity copper ion transport